{
  "term_label": "negative regulation of ERK1 and ERK2 cascade",
  "gene_symbol": "TNIP1",
  "term_id": "GO:0070373",
  "gene_name": "TNFAIP3-interacting protein 1",
  "gene": "UniProtKB:Q15025"
}